sphingomyelin phosphodiesterase activator activity [GO:0016230] (molecular function) Sources: GOC:ai Definition: Binds to and increases the activity of the enzyme sphingomyelin phosphodiesterase. Relationships: is a type of GO:0016004; positively regulates GO:0004767 Also known as: neutral sphingomyelinase activator